{
  "gene_name": "RAC-beta serine_threonine-protein kinase",
  "gene_symbol": "AKT2",
  "term_label": "positive regulation of blood vessel endothelial cell migration",
  "term_id": "GO:0043536",
  "gene": "UniProtKB:P31751"
}